L-leucine binding [GO:0070728] (molecular function) Relationships: is a type of amino acid binding [GO:0016597]; is a type of GO:0031406; is a type of cation binding [GO:0043169] Also known as: Leu binding, leucine binding Sources: GOC:BHF, GOC:mah Definition: Binding to L-leucine, 2-amino-4-methylpentanoic acid.